{
  "term_label": "endoplasmic reticulum",
  "gene_name": "E3 ubiquitin-protein ligase AMFR",
  "term_id": "GO:0005783",
  "gene_symbol": "AMFR",
  "gene": "UniProtKB:Q9UKV5"
}